{
  "gene_symbol": "HUWE1",
  "term_id": "GO:0006284",
  "gene": "UniProtKB:Q7Z6Z7",
  "term_label": "base-excision repair",
  "gene_name": "E3 ubiquitin-protein ligase HUWE1"
}